regulation of synapse maturation [GO:0090128] (biological process) Subtypes: positive regulation of synapse maturation [GO:0090129], negative regulation of synapse maturation [GO:2000297] Definition: Any process that modulates the extent of synapse maturation, the process that organizes a synapse so that it attains its fully functional state. Relationships: is a type of regulation of developmental process [GO:0050793]; is a type of regulation of synapse organization [GO:0050807]; regulates synapse maturation [GO:0060074] Sources: GOC:ascb_2009, GOC:dph, GOC:tb